{
  "gene": "UniProtKB:Q8N9X5",
  "term_label": "Unknown biological process",
  "gene_symbol": "LINC02912",
  "term_id": "UNKNOWN:0002",
  "gene_name": "Putative protein encoded by LINC02912"
}